{
  "gene_name": "SLIT-ROBO Rho GTPase-activating protein 3",
  "term_label": "negative regulation of cell migration",
  "gene_symbol": "SRGAP3",
  "term_id": "GO:0030336",
  "gene": "UniProtKB:O43295"
}